glucose catabolic process to butyrate [GO:0030645] (biological process) Sources: ISBN:0198506732 Also known as: butyrate fermentation, glucose fermentation to butyrate Relationships: is a type of glucose catabolic process [GO:0006007]; is a type of fermentation [GO:0006113]; is a type of butyrate metabolic process [GO:0019605] Definition: The anaerobic chemical reactions and pathways resulting in the breakdown of glucose, with the production of acetic acid, butyric acid, carbon dioxide (CO2), and dihydrogen; effected by some saccharolytic species of Clostridium, e.g. C. butyricum.